{
  "term_id": "UNKNOWN:0002",
  "term_label": "Unknown biological process",
  "gene": "UniProtKB:Q3ZCW2",
  "gene_symbol": "LGALSL",
  "gene_name": "Galectin-related protein"
}